{
  "term_id": "GO:0016020",
  "term_label": "membrane",
  "gene": "UniProtKB:Q93084",
  "gene_name": "Sarcoplasmic_endoplasmic reticulum calcium ATPase 3",
  "gene_symbol": "ATP2A3"
}